{
  "term_id": "GO:0044323",
  "term_label": "retinoic acid-responsive element binding",
  "gene": "UniProtKB:P48443",
  "gene_symbol": "RXRG",
  "gene_name": "Retinoic acid receptor RXR-gamma"
}